{
  "gene_name": "Bcl-2-like protein 2",
  "term_label": "intrinsic apoptotic signaling pathway in response to DNA damage",
  "term_id": "GO:0008630",
  "gene_symbol": "BCL2L2",
  "gene": "UniProtKB:Q92843"
}